branch elongation involved in ureteric bud branching [GO:0060681] (biological process) Definition: The growth of a branch of the ureteric bud along its axis. Relationships: is a type of branch elongation of an epithelium [GO:0060602]; is part of branching involved in ureteric bud morphogenesis [GO:0001658]; is part of GO:0060677 References: PMID:16916378 Sources: GOC:dph Regulation: regulated by regulation of branch elongation involved in ureteric bud branching [GO:0072095]; negatively regulated by negative regulation of branch elongation involved in ureteric bud branching [GO:0072096]